{
  "gene_name": "Adhesion G protein-coupled receptor B3",
  "term_label": "neuron remodeling",
  "term_id": "GO:0016322",
  "gene_symbol": "ADGRB3",
  "gene": "UniProtKB:O60242"
}